{
  "gene_symbol": "CES3",
  "gene_name": "Carboxylesterase 3",
  "term_id": "UNKNOWN:0002",
  "gene": "UniProtKB:Q6UWW8",
  "term_label": "Unknown biological process"
}